regulation of intrinsic apoptotic signaling pathway in response to osmotic stress by p53 class mediator [GO:1902238] (biological process) Relationships: is a type of regulation of intrinsic apoptotic signaling pathway in response to osmotic stress [GO:1902218]; is_a regulation of intrinsic apoptotic signaling pathway by p53 class mediator [GO:1902253]; regulates intrinsic apoptotic signaling pathway in response to osmotic stress by p53 class mediator [GO:1990127] Definition: Any process that modulates the frequency, rate or extent of intrinsic apoptotic signaling pathway in response to osmotic stress by p53 class mediator. Subtypes: negative regulation of intrinsic apoptotic signaling pathway in response to osmotic stress by p53 class mediator [GO:1902239], positive regulation of intrinsic apoptotic signaling pathway in response to osmotic stress by p53 class mediator [GO:1902240] References: PMID:16571598 Sources: GOC:TermGenie, GOC:krc, GOC:mtg_apoptosis